positive regulation of T-helper 17 cell lineage commitment [GO:2000330] (biological process) Also known as: positive regulation of T-helper 17 cell fate commitment, positive regulation of Th17 cell lineage commitment, positive regulation of Th17 fate commitment Relationships: is a type of positive regulation of cell fate commitment [GO:0010455]; is a type of positive regulation of T-helper 17 cell differentiation [GO:2000321]; is_a regulation of T-helper 17 cell lineage commitment [GO:2000328]; positively regulates T-helper 17 cell lineage commitment [GO:0072540] Definition: Any process that activates or increases the frequency, rate or extent of T-helper 17 cell lineage commitment. Sources: GOC:BHF, GOC:mah